brassinosteroid mediated signaling pathway [GO:0009742] (biological process) References: PMID:16699538 Sources: GOC:sm Definition: The series of molecular signals mediated by the detection of brassinosteroid. Regulation: regulated by GO:1900457; negatively regulated by negative regulation of brassinosteroid mediated signaling pathway [GO:1900458]; positively regulated by GO:1900459 Relationships: is a type of cell surface receptor signaling pathway [GO:0007166]; is a type of GO:0043401; is part of cellular response to brassinosteroid stimulus [GO:0071367] Also known as: brassinosteroid mediated signalling